{
  "term_id": "GO:0030864",
  "term_label": "cortical actin cytoskeleton",
  "gene_name": "Melanophilin",
  "gene_symbol": "MLPH",
  "gene": "UniProtKB:Q9BV36"
}